regulation of Rap protein signal transduction [GO:0032487] (biological process) Relationships: is a type of regulation of small GTPase mediated signal transduction [GO:0051056]; regulates GO:0032486 Definition: Any process that modulates the frequency, rate or extent of Rap protein signal transduction. Sources: GOC:mah